macropinocytosis involved in viral entry into host cell [GO:0075510] (biological process) Relationships: is a type of endocytosis involved in viral entry into host cell [GO:0075509] Definition: Any macropinocytosis that is involved in the uptake of a virus into a host cell. References: PMID:17077125, PMID:19404330 Sources: GOC:jl, GOC:sp, VZ:800 Also known as: viral entry into host cell via macropinocytosis